{
  "gene_name": "WD repeat-containing protein 19",
  "term_id": "GO:0060271",
  "gene_symbol": "WDR19",
  "gene": "UniProtKB:Q8NEZ3",
  "term_label": "cilium assembly"
}